{
  "term_label": "nucleus",
  "term_id": "GO:0005634",
  "gene": "UniProtKB:O95948",
  "gene_name": "One cut domain family member 2",
  "gene_symbol": "ONECUT2"
}